N-glycan processing to lysosome [GO:0016256] (biological process) References: PMID:35536965 Definition: The modification of high-mannose N-glycans by UDP-N-acetylglucosamine-lysosomal-enzyme N-acetylglucosaminephosphotransferase and the subsequent removal of the N-acetylglucosamine residues yielding mannose-6-P that occurs in the ER-Golgi apparatus to N-glycans destined for the lysosome. Relationships: is a type of N-glycan processing [GO:0006491]; is part of protein targeting to lysosome [GO:0006622]